{
  "gene_symbol": "ADAM30",
  "term_label": "male gonad development",
  "gene": "UniProtKB:Q9UKF2",
  "gene_name": "Disintegrin and metalloproteinase domain-containing protein 30",
  "term_id": "GO:0008584"
}